{
  "term_label": "NuA4 histone acetyltransferase complex",
  "gene_name": "Putative male-specific lethal-3 protein-like 2",
  "gene": "UniProtKB:P0C860",
  "gene_symbol": "MSL3B",
  "term_id": "GO:0035267"
}